{
  "gene_name": "Receptor activity-modifying protein 3",
  "term_label": "receptor complex",
  "gene_symbol": "RAMP3",
  "gene": "UniProtKB:O60896",
  "term_id": "GO:0043235"
}